{
  "gene_name": "Claudin-10",
  "gene_symbol": "CLDN10",
  "term_label": "paracellular tight junction channel activity",
  "gene": "UniProtKB:P78369",
  "term_id": "GO:0160187"
}